pyrimidine deoxyribonucleotide salvage [GO:0010139] (biological process) Relationships: is a type of GO:0009221; is a type of pyrimidine nucleotide salvage [GO:0032262] Subtypes: dCMP salvage [GO:0006239], dTMP salvage [GO:0036198] Definition: The pathway by which pyrimidine bases or pyrimidine deoxyribonucleotides from pyrimidine nucleotide breakdown are converted back to pyrimidine deoxyribonucleotides. The salvage pathway is important where there is no de novo pyrimidine deoxyribonucleotide biosynthesis. Sources: GOC:pz